inferior olivary nucleus structural organization [GO:0021716] (biological process) Relationships: is_a anatomical structure arrangement [GO:0048532]; BFO_0000050 medulla oblongata structural organization [GO:0021581]; is part of GO:0021714 Definition: The process that contributes to the act of creating the structural organization of the inferior olivary nucleus structure. The inferior olivary nucleus is a capsule-shaped structure in the ventral medulla located just lateral and dorsal to the medullary pyramids. Neurons in the inferior olivary nucleus are the source of climbing fiber input to the cerebellar cortex; these neurons have been implicated in various functions, such as learning and timing of movements. Also known as: inferior olivary nucleus structural organisation, inferior olive structural organization Sources: GOC:cls, GOC:dgh, GOC:dph, GOC:jid, GO_REF:0000021